protein processing [GO:0016485] (biological process) Relationships: is a type of proteolysis [GO:0006508]; is a type of protein maturation [GO:0051604] Also known as: protein maturation by peptide bond cleavage, protein maturation by peptide bond hydrolysis, peptidolysis during protein maturation, protein maturation by proteolysis Definition: Any protein maturation process achieved by the cleavage of a peptide bond or bonds within a protein. Protein maturation is the process leading to the attainment of the full functional capacity of a protein. Regulation: positively regulated by GO:0010954; RO_0002212 by GO:0010955; regulated by GO:0070613 Sources: GOC:curators, GOC:jl, GOC:jsg Subtypes: activation of plasma proteins involved in acute inflammatory response [GO:0002541], signal peptide processing [GO:0006465], vacuolar protein processing [GO:0006624], protein autoprocessing [GO:0016540], protein splicing [GO:0030908], zymogen activation [GO:0031638], mitochondrial protein processing [GO:0034982], Notch receptor processing, ligand-independent [GO:0035334], CAAX-box protein processing [GO:0071586], dibasic protein processing [GO:0090472], signaling receptor ligand precursor processing [GO:0140448], protein processing in phagocytic vesicle [GO:1900756]